{
  "gene": "UniProtKB:Q8N6M5",
  "term_label": "Unknown biological process",
  "term_id": "UNKNOWN:0002",
  "gene_name": "Probable inactive allantoicase",
  "gene_symbol": "ALLC"
}